{
  "term_id": "GO:0046899",
  "term_label": "nucleoside triphosphate adenylate kinase activity",
  "gene": "UniProtKB:Q9UIJ7",
  "gene_name": "GTP:AMP phosphotransferase AK3, mitochondrial",
  "gene_symbol": "AK3"
}